{
  "term_label": "serine-type endopeptidase activity",
  "gene": "UniProtKB:Q9UKR3",
  "term_id": "GO:0004252",
  "gene_symbol": "KLK13",
  "gene_name": "Kallikrein-13"
}